{
  "gene": "UniProtKB:O15014",
  "term_id": "GO:0006357",
  "gene_name": "Zinc finger protein 609",
  "term_label": "regulation of transcription by RNA polymerase II",
  "gene_symbol": "ZNF609"
}